{
  "gene_symbol": "CAMTA1",
  "term_id": "GO:0003712",
  "term_label": "transcription coregulator activity",
  "gene": "UniProtKB:Q9Y6Y1",
  "gene_name": "Calmodulin-binding transcription activator 1"
}